{
  "term_label": "skeletal muscle contraction",
  "term_id": "GO:0003009",
  "gene": "UniProtKB:P07510",
  "gene_name": "Acetylcholine receptor subunit gamma",
  "gene_symbol": "CHRNG"
}